{
  "gene_name": "Inosine triphosphate pyrophosphatase",
  "gene": "UniProtKB:Q9BY32",
  "term_label": "nucleoside triphosphate diphosphatase activity",
  "term_id": "GO:0047429",
  "gene_symbol": "ITPA"
}